{
  "gene_name": "Class A basic helix-loop-helix protein 9",
  "gene": "UniProtKB:Q7RTU4",
  "gene_symbol": "BHLHA9",
  "term_id": "UNKNOWN:0003",
  "term_label": "Unknown cellular component"
}